protein localization to microtubule [GO:0035372] (biological process) Regulation: regulated by regulation of protein localization to microtubule [GO:1902816]; negatively regulated by negative regulation of protein localization to microtubule [GO:1902817] Relationships: is a type of protein localization to microtubule cytoskeleton [GO:0072698] Sources: GOC:bf, GOC:lb Definition: A process in which a protein is transported to, or maintained at, a microtubule. Also known as: protein localisation to microtubule Subtypes: protein localization to spindle microtubule [GO:1902889], protein localization to microtubule end [GO:1905725], protein localization to cytoplasmic microtubule [GO:1905755]